phosphoketolase activity [GO:0050193] (molecular function) Also known as: D-xylulose-5-phosphate D-glyceraldehyde-3-phosphate-lyase (adding phosphate; acetyl-phosphate-forming), D-xylulose-5-phosphate D-glyceraldehyde-3-phosphate-lyase (phosphate-acetylating) activity, xylulose-5-phosphate phosphoketolase activity Definition: Catalysis of the reaction: D-xylulose 5-phosphate + phosphate = acetyl phosphate + D-glyceraldehyde 3-phosphate + H2O. Relationships: is a type of aldehyde-lyase activity [GO:0016832] Sources: EC:4.1.2.9, MetaCyc:PHOSPHOKETOLASE-RXN